{
  "gene": "UniProtKB:P53634",
  "term_id": "GO:0004197",
  "gene_name": "Dipeptidyl peptidase 1",
  "term_label": "cysteine-type endopeptidase activity",
  "gene_symbol": "CTSC"
}